{
  "gene_name": "BET1-like protein",
  "term_label": "SNAP receptor activity",
  "term_id": "GO:0005484",
  "gene": "UniProtKB:Q9NYM9",
  "gene_symbol": "BET1L"
}